{
  "term_label": "Unknown cellular component",
  "gene_symbol": "TNIP3",
  "gene_name": "TNFAIP3-interacting protein 3",
  "term_id": "UNKNOWN:0003",
  "gene": "UniProtKB:Q96KP6"
}